{
  "gene_symbol": "PANK2",
  "gene_name": "Pantothenate kinase 2, mitochondrial",
  "term_label": "pantothenate kinase activity",
  "term_id": "GO:0004594",
  "gene": "UniProtKB:Q9BZ23"
}